{
  "gene_symbol": "IFNA21",
  "term_label": "humoral immune response",
  "gene_name": "Interferon alpha-21",
  "term_id": "GO:0006959",
  "gene": "UniProtKB:P01568"
}